{
  "term_label": "Unknown biological process",
  "gene": "UniProtKB:Q969T3",
  "gene_symbol": "SNX21",
  "term_id": "UNKNOWN:0002",
  "gene_name": "Sorting nexin-21"
}